{
  "gene_symbol": "COMMD1",
  "term_id": "GO:2000009",
  "gene_name": "COMM domain-containing protein 1",
  "term_label": "negative regulation of protein localization to cell surface",
  "gene": "UniProtKB:Q8N668"
}